{
  "term_id": "GO:0042585",
  "gene_name": "Protein STPG4",
  "term_label": "germinal vesicle",
  "gene": "UniProtKB:Q8N801",
  "gene_symbol": "STPG4"
}